{
  "gene_symbol": "OR51A4",
  "term_label": "Unknown biological process",
  "gene": "UniProtKB:Q8NGJ6",
  "term_id": "UNKNOWN:0002",
  "gene_name": "Olfactory receptor 51A4"
}